{
  "term_id": "GO:0030175",
  "gene": "UniProtKB:P26038",
  "gene_symbol": "MSN",
  "gene_name": "Moesin",
  "term_label": "filopodium"
}